specification of floral organ identity [GO:0010093] (biological process) Subtypes: specification of carpel identity [GO:0010094], specification of petal identity [GO:0010095], specification of sepal identity [GO:0010096], specification of stamen identity [GO:0010097] Sources: GOC:tb Definition: The process in which the identity of a floral organ primordium is specified. Identity is considered to be the aggregate of characteristics by which a structure is recognized. Relationships: is a type of GO:0003006; is a type of specification of plant organ identity [GO:0090701]; is part of GO:0048449